{
  "term_id": "GO:0046597",
  "gene_name": "Interferon-induced transmembrane protein 1",
  "term_label": "host-mediated suppression of symbiont invasion",
  "gene_symbol": "IFITM1",
  "gene": "UniProtKB:P13164"
}